{
  "term_label": "intracellular signal transduction",
  "gene": "UniProtKB:Q9H9A6",
  "term_id": "GO:0035556",
  "gene_name": "Leucine-rich repeat-containing protein 40",
  "gene_symbol": "LRRC40"
}